{
  "gene_symbol": "KCNMB4",
  "gene_name": "Calcium-activated potassium channel subunit beta-4",
  "term_label": "voltage-gated potassium channel complex",
  "gene": "UniProtKB:Q86W47",
  "term_id": "GO:0008076"
}